{
  "term_id": "UNKNOWN:0003",
  "gene": "UniProtKB:Q13201",
  "gene_name": "Multimerin-1",
  "gene_symbol": "MMRN1",
  "term_label": "Unknown cellular component"
}